{
  "term_id": "GO:0005814",
  "term_label": "centriole",
  "gene": "UniProtKB:Q6ZU80",
  "gene_name": "Centrosomal protein of 128 kDa",
  "gene_symbol": "CEP128"
}